positive regulation of mast cell cytokine production [GO:0032765] (BP) Definition: Any process that activates or increases the frequency, rate, or extent of mast cell cytokine production. Also known as: up regulation of mast cell cytokine production, up-regulation of mast cell cytokine production, upregulation of mast cell cytokine production, activation of mast cell cytokine production, stimulation of mast cell cytokine production Sources: GOC:mah Relationships: is_a regulation of mast cell cytokine production [GO:0032763]; is a type of positive regulation of myeloid leukocyte cytokine production involved in immune response [GO:0061081]; positively regulates mast cell cytokine production [GO:0032762]